{
  "gene_symbol": "GLOD5",
  "gene": "UniProtKB:A6NK44",
  "gene_name": "Glyoxalase domain-containing protein 5",
  "term_id": "UNKNOWN:0003",
  "term_label": "Unknown cellular component"
}